negative regulation of ion transmembrane transporter activity [GO:0032413] (biological process) Also known as: down regulation of ion transporter activity, down-regulation of ion transporter activity, downregulation of ion transporter activity, negative regulation of ion transporter activity, inhibition of ion transporter activity Sources: GOC:mah, GOC:tb Definition: Any process that stops or reduces the activity of an ion transporter. Relationships: is a type of regulation of transmembrane transporter activity [GO:0022898]; is a type of GO:0032410; is a type of negative regulation of monoatomic ion transmembrane transport [GO:0034766]; negatively regulates monoatomic ion transmembrane transporter activity [GO:0015075] Subtypes: negative regulation of anion channel activity [GO:0010360], negative regulation of potassium ion transmembrane transporter activity [GO:1901017], GO:1901020, negative regulation of NMDA glutamate receptor activity [GO:1904782]